negative regulation of small intestine smooth muscle contraction [GO:1904348] (biological process) Definition: Any process that stops, prevents or reduces the frequency, rate or extent of small intestine smooth muscle contraction. References: PMID:11991626 Sources: GOC:TermGenie, GO_REF:0000058 Relationships: is a type of negative regulation of gastro-intestinal system smooth muscle contraction [GO:1904305]; is a type of regulation of small intestine smooth muscle contraction [GO:1904347]; RO_0002212 small intestine smooth muscle contraction [GO:1990770] Also known as: down regulation of small intestine smooth muscle contraction, down-regulation of small intestine smooth muscle contraction, downregulation of small intestine smooth muscle contraction, inhibition of small intestine smooth muscle contraction